{
  "term_label": "maintenance of presynaptic active zone structure",
  "gene": "UniProtKB:O15083",
  "gene_name": "ERC protein 2",
  "term_id": "GO:0048790",
  "gene_symbol": "ERC2"
}